{
  "gene_name": "TSC22 domain family protein 3",
  "term_id": "UNKNOWN:0001",
  "term_label": "Unknown molecular function",
  "gene_symbol": "TSC22D3",
  "gene": "UniProtKB:Q99576"
}